{
  "gene_symbol": "LRRK2",
  "gene_name": "Leucine-rich repeat serine_threonine-protein kinase 2",
  "term_id": "GO:0007029",
  "term_label": "endoplasmic reticulum organization",
  "gene": "UniProtKB:Q5S007"
}